{
  "gene": "UniProtKB:Q9UKL4",
  "gene_name": "Gap junction delta-2 protein",
  "gene_symbol": "GJD2",
  "term_label": "cell-cell signaling",
  "term_id": "GO:0007267"
}